UDP-glucosylation [GO:0097359] (biological process) Sources: GOC:al Definition: The covalent attachment of a UDP-glucose residue to a substrate molecule. Relationships: is a type of UDP-alpha-D-glucose metabolic process [GO:0006011]